{
  "gene_symbol": "INPP5K",
  "gene_name": "Inositol polyphosphate 5-phosphatase K",
  "term_id": "GO:0004439",
  "term_label": "phosphatidylinositol-4,5-bisphosphate 5-phosphatase activity",
  "gene": "UniProtKB:Q9BT40"
}